{
  "gene_symbol": "TSLP",
  "gene_name": "Thymic stromal lymphopoietin",
  "term_id": "GO:0032736",
  "term_label": "positive regulation of interleukin-13 production",
  "gene": "UniProtKB:Q969D9"
}